{
  "gene_symbol": "RAB33B",
  "term_label": "regulation of exocytosis",
  "gene": "UniProtKB:Q9H082",
  "term_id": "GO:0017157",
  "gene_name": "Ras-related protein Rab-33B"
}